{
  "gene_name": "Postacrosomal sheath WW domain-binding protein",
  "gene_symbol": "WBP2NL",
  "term_label": "transcription coactivator activity",
  "term_id": "GO:0003713",
  "gene": "UniProtKB:Q6ICG8"
}